{
  "term_id": "UNKNOWN:0001",
  "gene_name": "Protein BTG1",
  "term_label": "Unknown molecular function",
  "gene_symbol": "BTG1",
  "gene": "UniProtKB:P62324"
}